{
  "gene_symbol": "FBXO43",
  "term_label": "negative regulation of meiotic nuclear division",
  "gene": "UniProtKB:Q4G163",
  "gene_name": "F-box only protein 43",
  "term_id": "GO:0045835"
}